{
  "gene_name": "Amiloride-sensitive amine oxidase [copper-containing]",
  "term_label": "diamine oxidase activity",
  "gene_symbol": "AOC1",
  "term_id": "GO:0052597",
  "gene": "UniProtKB:P19801"
}